positive regulation of cardiac muscle cell contraction [GO:0106134] (biological process) Relationships: is a type of GO:0086004; is a type of positive regulation of actin filament-based movement [GO:1903116]; positively regulates cardiac muscle cell contraction [GO:0086003] Subtypes: positive regulation of ventricular cardiac muscle cell action potential [GO:1903947] References: PMID:19525381 Definition: Any process that activates or increases the frequency, rate or extent of cardiac muscle cell contraction.